insulin-like growth factor ternary complex [GO:0042567] (cellular component) Also known as: IGF ternary complex References: PMID:12239079 Sources: GOC:jl Definition: A complex of three proteins, which in animals is approximately 150kDa and consists of the insulin-like growth factor (IGF), the insulin-like growth factor binding protein-3 (IGFBP-3), or -5 (IGFBP-5) and an acid-labile subunit (ALS). The complex plays a role in growth and development. Relationships: is a type of insulin-like growth factor binding protein complex [GO:0016942]